{
  "gene_symbol": "KCNK2",
  "term_label": "plasma membrane",
  "gene_name": "Potassium channel subfamily K member 2",
  "term_id": "GO:0005886",
  "gene": "UniProtKB:O95069"
}